{
  "gene": "UniProtKB:Q7L590",
  "gene_symbol": "MCM10",
  "gene_name": "Protein MCM10 homolog",
  "term_label": "DNA replication initiation",
  "term_id": "GO:0006270"
}